{
  "gene": "UniProtKB:Q02094",
  "term_id": "GO:0072488",
  "gene_symbol": "RHAG",
  "term_label": "ammonium transmembrane transport",
  "gene_name": "Ammonium transporter Rh type A"
}